cotranscriptional mitochondrial rRNA nucleotide insertion [GO:0002110] (biological process) Relationships: is a type of GO:0000154; is_a RNA nucleotide insertion [GO:0070705] References: PMID:8306965 Sources: GOC:curators, ISBN:1555811337 Definition: The insertion of one or two non-coded nucleotides during the transcription of a mitochondrial rRNA. Such additions are known to occur in myxomycetes such as Physarum, Didymium, and Stemonitis.